{
  "term_label": "ATPase-coupled transmembrane transporter activity",
  "gene_symbol": "ABCD3",
  "gene_name": "ATP-binding cassette sub-family D member 3",
  "gene": "UniProtKB:P28288",
  "term_id": "GO:0042626"
}